{
  "term_label": "microtubule plus-end binding",
  "gene": "UniProtKB:Q15691",
  "term_id": "GO:0051010",
  "gene_symbol": "MAPRE1",
  "gene_name": "Microtubule-associated protein RP_EB family member 1"
}